{
  "gene_name": "Phosphatidylinositol 5-phosphate 4-kinase type-2 beta",
  "term_label": "plasma membrane",
  "gene": "UniProtKB:P78356",
  "gene_symbol": "PIP4K2B",
  "term_id": "GO:0005886"
}